{
  "gene": "UniProtKB:P48065",
  "gene_name": "Sodium- and chloride-dependent betaine transporter",
  "term_id": "GO:0035725",
  "term_label": "sodium ion transmembrane transport",
  "gene_symbol": "SLC6A12"
}